{
  "gene_name": "D-dopachrome decarboxylase",
  "gene_symbol": "DDT",
  "term_label": "extracellular space",
  "gene": "UniProtKB:P30046",
  "term_id": "GO:0005615"
}